negative regulation of CAMKK-AMPK signaling cascade [GO:1905290] (biological process) Relationships: is a type of negative regulation of calcium-mediated signaling [GO:0050849]; is a type of GO:1905289; negatively regulates CAMKK-AMPK signaling cascade [GO:0061762] References: PMID:22128786 Sources: GOC:TermGenie, GO_REF:0000058 Definition: Any process that stops, prevents or reduces the frequency, rate or extent of CAMKK-AMPK signaling cascade. Also known as: down regulation of CAMKK-AMPK signaling cascade, down-regulation of CAMKK-AMPK signaling cascade, downregulation of CAMKK-AMPK signaling cascade, inhibition of CAMKK-AMPK signaling cascade, down regulation of stress-activated AMP-activated protein kinase signaling cascade, down-regulation of stress-activated AMP-activated protein kinase signaling cascade, downregulation of stress-activated AMP-activated protein kinase signaling cascade, inhibition of stress-activated AMP-activated protein kinase signaling cascade, negative regulation of stress-activated AMP-activated protein kinase signaling cascade